corticospinal neuron axon guidance through spinal cord [GO:0021972] (biological process) Relationships: is a type of axon guidance [GO:0007411]; is part of GO:0021966 Definition: The process in which the migration of an axon growth cone of a pyramidal cell that is part of the corticospinal tract is directed after decussation through the spinal cord in response to a combination of attractive and repulsive cues. Also known as: corticospinal neuron axon pathfinding through spinal cord References: PMID:9878731 Sources: GOC:cls, GOC:dgh, GOC:dph, GOC:jid, GO_REF:0000021